{
  "term_id": "GO:0005737",
  "gene_name": "G protein-coupled receptor kinase 5",
  "gene_symbol": "GRK5",
  "gene": "UniProtKB:P34947",
  "term_label": "cytoplasm"
}